{
  "term_label": "mitochondrion",
  "gene_name": "Phosphoenolpyruvate carboxykinase [GTP], mitochondrial",
  "gene": "UniProtKB:Q16822",
  "term_id": "GO:0005739",
  "gene_symbol": "PCK2"
}